p-cumate catabolic process [GO:1901782] (biological process) References: PMID:8631713 Sources: GOC:TermGenie, GOC:yaf, MetaCyc:PWY-5273, UniPathway:UPA00937 Also known as: p-cumate breakdown, p-cumate catabolism, p-cumate degradation Definition: The chemical reactions and pathways resulting in the breakdown of p-cumate. Relationships: is_a benzene-containing compound metabolic process [GO:0042537]; is a type of monocarboxylic acid catabolic process [GO:0072329]